{
  "term_id": "UNKNOWN:0003",
  "gene": "UniProtKB:Q6S9Z5",
  "gene_name": "Zinc finger protein 474",
  "term_label": "Unknown cellular component",
  "gene_symbol": "ZNF474"
}